{
  "gene_name": "Zinc finger protein 79",
  "gene": "UniProtKB:Q15937",
  "term_label": "nucleus",
  "gene_symbol": "ZNF79",
  "term_id": "GO:0005634"
}